{
  "term_label": "axon guidance",
  "gene_name": "Pleckstrin homology domain-containing family G member 4B",
  "gene": "UniProtKB:Q96PX9",
  "term_id": "GO:0007411",
  "gene_symbol": "PLEKHG4B"
}